tolerance induction in nasopharyngeal-associated lymphoid tissue [GO:0002400] (biological process) Also known as: tolerance induction in NALT, nasal tolerance Definition: Tolerance induction taking place in the nasopharyngeal-associated lymphoid tissue (NALT). Sources: GOC:jal, ISBN:0781735149 Relationships: is a type of GO:0002394; is a type of immune response in nasopharyngeal-associated lymphoid tissue [GO:0002395]